{
  "gene_symbol": "PTPN13",
  "gene": "UniProtKB:Q12923",
  "term_id": "GO:0036312",
  "term_label": "phosphatidylinositol 3-kinase regulatory subunit binding",
  "gene_name": "Tyrosine-protein phosphatase non-receptor type 13"
}